co-transcriptional lncRNA 3' end processing, cleavage and polyadenylation pathway [GO:0180034] (biological process) References: PMID:31276588 Relationships: is a type of GO:0180012; is a type of lncRNA processing [GO:0180035] Definition: Any process involved in transcription termination-coupled 3' processing of RNA polymerase II lncRNA transcripts by the 3' end cleavage and addition of a poly(A) tail. Also known as: lncRNA 3' end processing, lncRNA 3'-end processing